{
  "term_id": "GO:0000981",
  "gene_name": "Signal transducer and activator of transcription 6",
  "gene": "UniProtKB:P42226",
  "gene_symbol": "STAT6",
  "term_label": "DNA-binding transcription factor activity, RNA polymerase II-specific"
}